{
  "gene_symbol": "SPIRE2",
  "gene_name": "Protein spire homolog 2",
  "term_id": "GO:0051639",
  "gene": "UniProtKB:Q8WWL2",
  "term_label": "actin filament network formation"
}